response to muscle stretch [GO:0035994] (biological process) References: PMID:14583192 Sources: GOC:BHF, GOC:vk Relationships: is a type of GO:0009612 Definition: Any process that results in a change in state or activity of a cell or an organism (in terms of movement, secretion, enzyme production, gene expression, etc.) as a result of a myofibril being extended beyond its slack length. Subtypes: detection of muscle stretch [GO:0035995]